cyclopeptine synthase activity [GO:0047671] (molecular function) Also known as: ATP:anthranilate adenylyltransferase activity, anthranilate adenylyltransferase activity Definition: Catalysis of the reaction: anthranilate + 2 ATP + L-phenylalanine + S-adenosyl-L-methionine = 2 AMP + cyclopeptine + 2 diphosphate + 2 H+ + S-adenosyl-L-homocysteine. Relationships: is a type of acid-amino acid ligase activity [GO:0016881] References: PMID:2995633 Sources: EC:6.3.2.40, RHEA:35091